{
  "gene_name": "S phase cyclin A-associated protein in the endoplasmic reticulum",
  "gene": "UniProtKB:Q9BY12",
  "gene_symbol": "SCAPER",
  "term_id": "UNKNOWN:0002",
  "term_label": "Unknown biological process"
}